regulation of cellular response to hypoxia [GO:1900037] (BP) Relationships: is a type of regulation of cellular response to stress [GO:0080135]; regulates cellular response to hypoxia [GO:0071456] Definition: Any process that modulates the frequency, rate or extent of cellular response to hypoxia. Sources: GOC:TermGenie, GOC:yaf Subtypes: negative regulation of cellular response to hypoxia [GO:1900038], positive regulation of cellular response to hypoxia [GO:1900039] Also known as: regulation of cellular response to hypoxic stress, regulation of cellular response to lowered oxygen tension